metaplastic ossification [GO:0036074] (BP) Relationships: is a type of direct ossification [GO:0036072] Definition: Direct ossification in which bone formation occurs as result of the direct transformation of non-bone cells into bone cells without cell division. Also known as: metaplasia Note: Some intramembranous ossification may also be classified as metaplastic; the former classifies based on tissue type location, and the latter based on mechanism/cell division. Sources: GO_REF:0000034